{
  "gene": "UniProtKB:Q8N9P6",
  "gene_symbol": "C9orf163",
  "term_label": "Unknown cellular component",
  "term_id": "UNKNOWN:0003",
  "gene_name": "Uncharacterized protein C9orf163"
}